{
  "gene_symbol": "SLF1",
  "gene": "UniProtKB:Q9BQI6",
  "term_label": "protein localization to site of double-strand break",
  "gene_name": "SMC5-SMC6 complex localization factor protein 1",
  "term_id": "GO:1990166"
}